positive regulation of acetylcholine biosynthetic process [GO:1905923] (biological process) Definition: Any process that activates or increases the frequency, rate or extent of acetylcholine biosynthetic process. References: PMID:20164328 Sources: GOC:TermGenie, GOC:aruk, GOC:bc, GO_REF:0000058 Also known as: positive regulation of acetylcholine anabolism, positive regulation of acetylcholine biosynthesis, positive regulation of acetylcholine formation, positive regulation of acetylcholine synthesis, up regulation of acetylcholine anabolism, up regulation of acetylcholine biosynthesis, up regulation of acetylcholine biosynthetic process, up regulation of acetylcholine formation, up regulation of acetylcholine synthesis, up-regulation of acetylcholine anabolism, up-regulation of acetylcholine biosynthesis, up-regulation of acetylcholine biosynthetic process, up-regulation of acetylcholine formation, up-regulation of acetylcholine synthesis, upregulation of acetylcholine anabolism, upregulation of acetylcholine biosynthesis, upregulation of acetylcholine biosynthetic process, upregulation of acetylcholine formation, upregulation of acetylcholine synthesis, activation of acetylcholine anabolism, activation of acetylcholine biosynthesis, activation of acetylcholine biosynthetic process, activation of acetylcholine formation, activation of acetylcholine synthesis Relationships: is a type of GO:0009891; is a type of positive regulation of acetylcholine metabolic process [GO:0060409]; is a type of GO:1905921; positively regulates acetylcholine biosynthetic process [GO:0008292]